{
  "gene_name": "Lysine-specific demethylase 5C",
  "gene_symbol": "KDM5C",
  "gene": "UniProtKB:P41229",
  "term_id": "GO:0000785",
  "term_label": "chromatin"
}